regulation of nucleotide biosynthetic process [GO:0030808] (biological process) Sources: GOC:mah Definition: Any process that modulates the frequency, rate or extent of the chemical reactions and pathways resulting in the formation of nucleotides. Relationships: is a type of regulation of nucleotide metabolic process [GO:0006140]; is a type of regulation of biosynthetic process [GO:0009889]; regulates nucleotide biosynthetic process [GO:0009165] Subtypes: negative regulation of nucleotide biosynthetic process [GO:0030809], positive regulation of nucleotide biosynthetic process [GO:0030810], regulation of purine nucleotide biosynthetic process [GO:1900371], regulation of pyrimidine nucleotide biosynthetic process [GO:1900397] Also known as: regulation of nucleotide anabolism, regulation of nucleotide biosynthesis, regulation of nucleotide formation, regulation of nucleotide synthesis